{
  "gene_symbol": "LIMS2",
  "term_id": "GO:2001046",
  "gene_name": "LIM and senescent cell antigen-like-containing domain protein 2",
  "term_label": "positive regulation of integrin-mediated signaling pathway",
  "gene": "UniProtKB:Q7Z4I7"
}